L-rhamnose isomerase activity [GO:0008740] (molecular function) Sources: RHEA:23160 Relationships: is a type of intramolecular oxidoreductase activity, interconverting aldoses and ketoses [GO:0016861] Also known as: L-rhamnose aldose-ketose-isomerase activity, L-rhamnose ketol-isomerase activity, rhamnose isomerase activity Definition: Catalysis of the reaction: L-rhamnose = L-rhamnulose.